{
  "gene_name": "N-acetylmuramoyl-L-alanine amidase",
  "term_id": "GO:0006955",
  "term_label": "immune response",
  "gene": "UniProtKB:Q96PD5",
  "gene_symbol": "PGLYRP2"
}